{
  "gene_symbol": "SLC22A4",
  "term_label": "quaternary ammonium group transport",
  "term_id": "GO:0015697",
  "gene": "UniProtKB:Q9H015",
  "gene_name": "Solute carrier family 22 member 4"
}